{
  "term_label": "ubiquitin-dependent endocytosis",
  "gene_symbol": "NEURL1B",
  "gene_name": "E3 ubiquitin-protein ligase NEURL1B",
  "term_id": "GO:0070086",
  "gene": "UniProtKB:A8MQ27"
}